{
  "gene_name": "Short-chain specific acyl-CoA dehydrogenase, mitochondrial",
  "gene": "UniProtKB:P16219",
  "term_id": "GO:0033539",
  "gene_symbol": "ACADS",
  "term_label": "fatty acid beta-oxidation using acyl-CoA dehydrogenase"
}